{
  "gene_name": "Forkhead box protein O1",
  "gene": "UniProtKB:Q12778",
  "term_label": "nucleus",
  "term_id": "GO:0005634",
  "gene_symbol": "FOXO1"
}